{
  "gene_name": "Cytospin-B",
  "term_label": "actin cytoskeleton organization",
  "term_id": "GO:0030036",
  "gene": "UniProtKB:Q5M775",
  "gene_symbol": "SPECC1"
}